{
  "gene": "UniProtKB:Q96SD1",
  "term_id": "GO:0006303",
  "gene_name": "Protein artemis",
  "gene_symbol": "DCLRE1C",
  "term_label": "double-strand break repair via nonhomologous end joining"
}